{
  "term_id": "UNKNOWN:0002",
  "term_label": "Unknown biological process",
  "gene": "UniProtKB:Q8IZT6",
  "gene_name": "Abnormal spindle-like microcephaly-associated protein",
  "gene_symbol": "ASPM"
}